{
  "gene_symbol": "STAB1",
  "term_id": "UNKNOWN:0003",
  "gene_name": "Stabilin-1",
  "gene": "UniProtKB:Q9NY15",
  "term_label": "Unknown cellular component"
}